{
  "gene": "UniProtKB:Q9H6K5",
  "term_label": "Unknown biological process",
  "gene_name": "Proline-rich protein 36",
  "gene_symbol": "PRR36",
  "term_id": "UNKNOWN:0002"
}